UDP-glucuronate decarboxylase activity [GO:0048040] (molecular function) Definition: Catalysis of the reaction: H+ + UDP-alpha-D-glucuronate = CO2 + UDP-alpha-D-xylose. Sources: EC:4.1.1.35, RHEA:23916 Relationships: is a type of carboxy-lyase activity [GO:0016831] Also known as: UDP-glucuronic acid decarboxylase activity, UDP-D-glucuronate carboxy-lyase (UDP-D-xylose-forming), UDP-D-glucuronate carboxy-lyase activity, UDPglucuronate decarboxylase activity, uridine-diphosphoglucuronate decarboxylase activity